{
  "term_label": "Unknown molecular function",
  "term_id": "UNKNOWN:0001",
  "gene": "UniProtKB:Q9BZ97",
  "gene_name": "Putative transcript Y 13 protein",
  "gene_symbol": "TTTY13"
}